lipopolysaccharide floppase activity [GO:0015437] (MF) Relationships: is a type of floppase activity [GO:0140328]; is part of GO:0015920 Also known as: ATPase-coupled intramembrane lipopolysaccharide transporter activity, ATP-dependent intramembrane lipopolysaccharide transporter activity, LPS-transporting ATPase activity, lipopolysaccharide floppase activity (cytosolic to exoplasmic leaflet), lipopolysaccharide-transporting ATPase activity Sources: EC:7.5.2.5 Definition: Enables the transfer of a lipopolysaccharide from the cytosolic to the exoplasmic leaflet of a membrane, using energy from the hydrolysis of ATP.